{
  "term_id": "GO:0005829",
  "gene_name": "Serine_threonine-protein phosphatase 2A catalytic subunit beta isoform",
  "gene_symbol": "PPP2CB",
  "term_label": "cytosol",
  "gene": "UniProtKB:P62714"
}